{
  "term_label": "anterior/posterior pattern specification",
  "term_id": "GO:0009952",
  "gene_symbol": "CRIPTO3",
  "gene": "UniProtKB:P51864",
  "gene_name": "Putative teratocarcinoma-derived growth factor 3"
}